response to interleukin-9 [GO:0071104] (BP) Also known as: response to IL-9 Definition: Any process that results in a change in state or activity of a cell or an organism (in terms of movement, secretion, enzyme production, gene expression, etc.) as a result of an interleukin-9 stimulus. Subtypes: cellular response to interleukin-9 [GO:0071355] Relationships: is a type of GO:0034097 Sources: GOC:mah, GOC:yaf